{
  "gene_name": "Small ribosomal subunit protein eS26",
  "gene_symbol": "RPS26",
  "term_id": "GO:0022627",
  "gene": "UniProtKB:P62854",
  "term_label": "cytosolic small ribosomal subunit"
}